{
  "term_id": "GO:0015629",
  "gene_name": "Gamma-parvin",
  "gene": "UniProtKB:Q9HBI0",
  "gene_symbol": "PARVG",
  "term_label": "actin cytoskeleton"
}